positive regulation of branchiomeric skeletal muscle development [GO:0014712] (biological process) Sources: GOC:mtg_muscle Relationships: is a type of GO:0014711; is a type of GO:0048643; RO_0002213 GO:0014707 Definition: Any process that activates, maintains or increases the frequency, rate or extent of branchiomeric skeletal muscle development. Branchiomeric skeletal muscle development is the process whose specific outcome is the progression of the branchiomeric skeletal muscle over time, from its formation to the mature structure.